intramolecular acyltransferase activity [GO:0016867] (molecular function) Subtypes: precorrin-8X methylmutase activity [GO:0016993], cobalt-precorrin-8 methylmutase activity [GO:0043778], GO:0050070, beta-galactosidase activity (lactose isomerization) [GO:0103033] Definition: Catalysis of the transfer of an acyl group from one position to another within a single molecule. Relationships: is a type of intramolecular transferase activity [GO:0016866] Also known as: intramolecular transferase activity, transferring acyl groups Sources: GOC:mah